{
  "gene_symbol": "C10orf67",
  "gene": "UniProtKB:Q8IYJ2",
  "term_id": "UNKNOWN:0002",
  "term_label": "Unknown biological process",
  "gene_name": "Uncharacterized protein C10orf67, mitochondrial"
}